{
  "term_label": "delayed rectifier potassium channel activity",
  "gene": "UniProtKB:P22460",
  "term_id": "GO:0005251",
  "gene_symbol": "KCNA5",
  "gene_name": "Potassium voltage-gated channel subfamily A member 5"
}